receptor clustering activity [GO:0141175] (molecular function) Definition: A protein-protein adaptor that acts as a platform for receptor clustering, often serving to amplify the sensitivity of a signaling response. References: PMID:19747931, PMID:21453460, PMID:33597156 Relationships: is a type of GO:0030674